{
  "gene": "UniProtKB:O00151",
  "gene_name": "PDZ and LIM domain protein 1",
  "term_label": "filamentous actin",
  "gene_symbol": "PDLIM1",
  "term_id": "GO:0031941"
}